{
  "gene_symbol": "WASH3P",
  "gene_name": "Putative WAS protein family homolog 3",
  "term_id": "GO:0032456",
  "gene": "UniProtKB:C4AMC7",
  "term_label": "endocytic recycling"
}